{
  "gene": "UniProtKB:Q04609",
  "term_label": "carboxypeptidase activity",
  "term_id": "GO:0004180",
  "gene_symbol": "FOLH1",
  "gene_name": "Glutamate carboxypeptidase 2"
}